{
  "gene_symbol": "RIOK2",
  "gene_name": "Serine_threonine-protein kinase RIO2",
  "gene": "UniProtKB:Q9BVS4",
  "term_id": "GO:0030490",
  "term_label": "maturation of SSU-rRNA"
}